{
  "term_label": "phosphatidylinositol-3,4,5-trisphosphate 3-phosphatase activity",
  "gene_name": "Putative tyrosine-protein phosphatase TPTE",
  "gene": "UniProtKB:P56180",
  "term_id": "GO:0016314",
  "gene_symbol": "TPTE"
}